vinylacetate caboxylester hydrolase activity [GO:0102197] (molecular function) References: PMID:19555778 Sources: GOC:pz Definition: Catalysis of the reaction: but-3-enoate + H2O = allyl alcohol + formate. Relationships: is a type of carboxylic ester hydrolase activity [GO:0052689]